positive regulation of mesonephros development [GO:0061213] (biological process) Subtypes: GO:0061297 Definition: Any process that increases the rate, frequency or extent of mesonephros development. Mesonephros development is the process whose specific outcome is the progression of the mesonephros over time, from its formation to the mature structure. The mesonephros is an organ that filters the blood and excretes the end products of body metabolism in the form of urine. Relationships: is a type of regulation of mesonephros development [GO:0061217]; is a type of GO:0090184; positively regulates mesonephros development [GO:0001823] Sources: GOC:mtg_kidney_jan10